{
  "term_id": "UNKNOWN:0003",
  "gene_name": "Radial spoke head 10 homolog B2",
  "term_label": "Unknown cellular component",
  "gene_symbol": "RSPH10B2",
  "gene": "UniProtKB:B2RC85"
}